{
  "gene_symbol": "LEMD1",
  "gene_name": "LEM domain-containing protein 1",
  "term_label": "Unknown cellular component",
  "term_id": "UNKNOWN:0003",
  "gene": "UniProtKB:Q68G75"
}